{
  "gene": "UniProtKB:Q8N1G4",
  "gene_name": "Leucine-rich repeat-containing protein 47",
  "gene_symbol": "LRRC47",
  "term_label": "Unknown biological process",
  "term_id": "UNKNOWN:0002"
}